galactarate metabolic process [GO:0019580] (biological process) Subtypes: galactarate biosynthetic process [GO:0046357], galactarate catabolic process [GO:0046392] Relationships: is_a dicarboxylic acid metabolic process [GO:0043648] Also known as: galactarate metabolism, mucic acid metabolic process, mucic acid metabolism, D-galactarate metabolic process, D-galactarate metabolism Sources: GOC:pr, ISBN:0198506732 Definition: The chemical reactions and pathways involving galactarate, an anion of galactaric acid, the meso-aldaric acid derived from both D- and L-galactose.